{
  "gene_symbol": "PALS2",
  "term_label": "Unknown biological process",
  "gene": "UniProtKB:Q9NZW5",
  "term_id": "UNKNOWN:0002",
  "gene_name": "Protein PALS2"
}